{
  "gene_name": "Lactotransferrin",
  "term_id": "GO:0005886",
  "term_label": "plasma membrane",
  "gene": "UniProtKB:P02788",
  "gene_symbol": "LTF"
}